cyclic-GMP-AMP transmembrane import across plasma membrane [GO:0140361] (biological process) Relationships: is a type of organic anion transport [GO:0015711]; is a type of GO:0015868; is a type of adenine nucleotide transport [GO:0051503]; is a type of cyclic nucleotide transport [GO:0070729]; is a type of import across plasma membrane [GO:0098739]; is a type of guanine nucleotide transmembrane transport [GO:1903790] Definition: The directed movement of cyclic-GMP-AMP from outside of a cell, across the plasma membrane and into the cytosol. References: PMID:31126740